{
  "term_label": "potassium ion import across plasma membrane",
  "term_id": "GO:1990573",
  "gene": "UniProtKB:Q9H2X9",
  "gene_symbol": "SLC12A5",
  "gene_name": "Solute carrier family 12 member 5"
}